{
  "gene_name": "Coiled-coil and C2 domain-containing protein 1B",
  "gene_symbol": "CC2D1B",
  "gene": "UniProtKB:Q5T0F9",
  "term_label": "nucleus",
  "term_id": "GO:0005634"
}